{
  "gene": "UniProtKB:P04004",
  "gene_symbol": "VTN",
  "term_label": "extracellular matrix binding",
  "term_id": "GO:0050840",
  "gene_name": "Vitronectin"
}